cardiac pacemaker cell differentiation [GO:0060920] (biological process) Sources: GOC:mtg_cardiac_conduct_nov11, GOC:mtg_heart Subtypes: GO:0060921, atrioventricular node cell differentiation [GO:0060922] Also known as: pacemaker cell differentiation Definition: The process in which a relatively unspecialized cell acquires specialized features of a pacemaker cell. Pacemaker cells are specialized cardiomyocytes that are responsible for regulating the timing of heart contractions. Relationships: is a type of cardiac muscle cell differentiation [GO:0055007]